{
  "gene_name": "NADH dehydrogenase [ubiquinone] 1 subunit C2",
  "gene_symbol": "NDUFC2",
  "term_id": "UNKNOWN:0001",
  "term_label": "Unknown molecular function",
  "gene": "UniProtKB:O95298"
}